{
  "gene_symbol": "CHTF18",
  "term_label": "nucleus",
  "term_id": "GO:0005634",
  "gene_name": "Chromosome transmission fidelity protein 18 homolog",
  "gene": "UniProtKB:Q8WVB6"
}